{
  "term_label": "nucleosome",
  "gene_name": "Histone H2A type 1-J",
  "gene": "UniProtKB:Q99878",
  "term_id": "GO:0000786",
  "gene_symbol": "H2AC14"
}